puromycin biosynthetic process [GO:0043638] (biological process) Definition: The chemical reactions and pathways resulting in the formation of puromycin, an aminonucleoside antibiotic that is a potent inhibitor of translation; produced by the bacterium Streptomyces alboniger. Relationships: is a type of GO:0017000; is a type of purine ribonucleoside biosynthetic process [GO:0046129] Sources: GOC:jl, Wikipedia:Puromycin